{
  "gene_symbol": "MBLAC2",
  "term_label": "Unknown cellular component",
  "gene_name": "Acyl-coenzyme A thioesterase MBLAC2",
  "term_id": "UNKNOWN:0003",
  "gene": "UniProtKB:Q68D91"
}